{
  "gene_symbol": "RERE",
  "term_label": "transcription corepressor activity",
  "gene": "UniProtKB:Q9P2R6",
  "gene_name": "Arginine-glutamic acid dipeptide repeats protein",
  "term_id": "GO:0003714"
}